{
  "gene_symbol": "HYDIN",
  "term_id": "GO:0005930",
  "gene_name": "Hydrocephalus-inducing protein homolog",
  "term_label": "axoneme",
  "gene": "UniProtKB:Q4G0P3"
}